{
  "gene_name": "glutathione transferase",
  "gene": "UniProtKB:A0A1W2PRG0",
  "term_id": "GO:0005737",
  "term_label": "cytoplasm",
  "gene_symbol": "GSTTP2"
}